behavior [GO:0007610] (biological process) References: PMID:20160973 Sources: GOC:ems, GOC:jl, ISBN:0395448956 Also known as: behavioral response to stimulus, behaviour, behavioural response to stimulus, single-organism behavior Relationships: is a type of GO:0032501 Note: 1. Note that this term is in the subset of terms that should not be used for direct gene product annotation. Instead, select a child term or, if no appropriate child term exists, please request a new term. Direct annotations to this term may be amended during annotation reviews.
2. While a broader definition of behavior encompassing plants and single cell organisms would be justified on the basis of some usage (see PMID:20160973 for discussion), GO uses a tight definition that limits behavior to animals and to responses involving the nervous system, excluding plant responses that GO classifies under development, and responses of unicellular organisms that has general classifications for covering the responses of cells in multicellular organisms (e.g. cell chemotaxis). Subtypes: GO:0001966, aggressive behavior [GO:0002118], GO:0002209, behavioral response to wounding [GO:0002210], learning or memory [GO:0007611], rhythmic behavior [GO:0007622], grooming behavior [GO:0007625], locomotory behavior [GO:0007626], feeding behavior [GO:0007631], GO:0007632, GO:0007635, mechanosensory behavior [GO:0007638], reproductive behavior [GO:0019098], adult behavior [GO:0030534], GO:0030537, host-seeking behavior [GO:0032537], social behavior [GO:0035176], hatching behavior [GO:0035187], exploration behavior [GO:0035640], thermosensory behavior [GO:0040040], GO:0042630, GO:0048266, behavioral response to nutrient [GO:0051780], general adaptation syndrome, behavioral process [GO:0051867], crying behavior [GO:0060273], foraging behavior [GO:0060756], GO:0061744, vocalization behavior [GO:0071625], olfactory sociosexual communication [GO:0120318] Definition: The internally coordinated responses (actions or inactions) of animals (individuals or groups) to internal or external stimuli, via a mechanism that involves nervous system activity. Regulation: positively regulated by positive regulation of behavior [GO:0048520]; negatively regulated by negative regulation of behavior [GO:0048521]; regulated by regulation of behavior [GO:0050795]